{
  "term_id": "GO:0031507",
  "gene_name": "Histone H2A-Bbd type 1",
  "term_label": "heterochromatin formation",
  "gene_symbol": "H2AB1",
  "gene": "UniProtKB:P0C5Y9"
}